{
  "term_id": "GO:0034341",
  "gene": "UniProtKB:O15205",
  "term_label": "response to type II interferon",
  "gene_symbol": "UBD",
  "gene_name": "Ubiquitin D"
}